vesicle targeting to fusome [GO:0045479] (biological process) Definition: The recruitment of vesicles to the fusome. The vesicles become the fusome tubule network and are necessary for the assembly of the fusome. References: PMID:9046244 Also known as: vesicle-fusome targeting Relationships: is a type of GO:0006903; is part of fusome organization [GO:0045478]